negative regulation of receptor internalization [GO:0002091] (biological process) Subtypes: GO:1904021 Also known as: down regulation of receptor internalization, down-regulation of receptor internalization, downregulation of receptor internalization, inhibition of receptor internalization Relationships: is a type of GO:0002090; is a type of GO:0048261; RO_0002212 receptor internalization [GO:0031623] Sources: GOC:hjd Definition: Any process that stops, prevents, or reduces the frequency, rate or extent of receptor internalization.